{
  "gene_name": "Zinc finger protein 12",
  "gene_symbol": "ZNF12",
  "term_id": "GO:0005634",
  "term_label": "nucleus",
  "gene": "UniProtKB:P17014"
}